positive regulation of mesenchymal cell apoptotic process involved in nephron morphogenesis [GO:0072041] (biological process) Sources: GOC:mtg_apoptosis, GOC:mtg_kidney_jan10 Also known as: positive regulation of mesenchymal stem cell apoptotic process involved in nephron morphogenesis, positive regulation of mesenchymal stem cell apoptosis involved in nephron morphogenesis Subtypes: positive regulation of mesenchymal cell apoptotic process involved in mesonephric nephron morphogenesis [GO:0061297], positive regulation of mesenchymal cell apoptotic process involved in metanephric nephron morphogenesis [GO:0072306] Relationships: is a type of regulation of mesenchymal cell apoptotic process involved in nephron morphogenesis [GO:0072039]; is a type of positive regulation of apoptotic process involved in morphogenesis [GO:1902339]; is_a GO:1904674; is_a positive regulation of mesenchymal cell apoptotic process [GO:2001055]; positively regulates mesenchymal stem cell maintenance involved in nephron morphogenesis [GO:0072038]; positively regulates mesenchymal cell apoptotic process involved in nephron morphogenesis [GO:1901145] Definition: Any process that increases the occurrence or rate of mesenchymal stem cell death by apoptotic process that contributes to the shaping of the nephron.